L-tryptophan catabolic process to acetyl-CoA [GO:0019442] (biological process) Relationships: is a type of acetyl-CoA metabolic process [GO:0006084]; is a type of L-tryptophan catabolic process [GO:0006569]; is a type of GO:0043605 Sources: GOC:go_curators Definition: The chemical reactions and pathways resulting in the breakdown of L-tryptophan into other compounds, including acetyl-CoA. Also known as: tryptophan breakdown to acetyl-CoA, tryptophan catabolic process to acetyl-CoA, tryptophan degradation to acetyl-CoA